decidualization [GO:0046697] (biological process) Relationships: is_a developmental process involved in reproduction [GO:0003006]; is a type of tissue development [GO:0009888]; is part of maternal placenta development [GO:0001893] References: PMID:11133685 Sources: ISBN:0721662544 Also known as: decidual cell reaction Definition: The cellular and vascular changes occurring in the endometrium of the pregnant uterus just after the onset of blastocyst implantation. This process involves the proliferation and differentiation of the fibroblast-like endometrial stromal cells into large, polyploid decidual cells that eventually form the maternal component of the placenta.